{
  "term_label": "RNA polymerase II cis-regulatory region sequence-specific DNA binding",
  "gene_name": "Zinc finger protein 324B",
  "term_id": "GO:0000978",
  "gene": "UniProtKB:Q6AW86",
  "gene_symbol": "ZNF324B"
}